regulation of post-embryonic development [GO:0048580] (biological process) Definition: Any process that modulates the frequency, rate or extent of post-embryonic development. Post-embryonic development is defined as the process whose specific outcome is the progression of the organism over time, from the completion of embryonic development to the mature structure. Sources: GOC:jid Relationships: is_a regulation of multicellular organismal development [GO:2000026]; regulates GO:0009791 Subtypes: GO:0009909, GO:0010099, regulation of vegetative phase change [GO:0010321], negative regulation of post-embryonic development [GO:0048581], positive regulation of post-embryonic development [GO:0048582], GO:0061062, regulation of seed development [GO:0080050], GO:0090256, regulation of pupariation [GO:0106023], regulation of thermomorphogenesis [GO:0140920], regulation of seedling development [GO:1900140], regulation of stomatal complex development [GO:2000038], regulation of post-embryonic root development [GO:2000069]